{
  "term_label": "flap-structured DNA binding",
  "gene": "UniProtKB:Q9Y2M0",
  "gene_name": "Fanconi-associated nuclease 1",
  "gene_symbol": "FAN1",
  "term_id": "GO:0070336"
}